{
  "term_label": "Unknown cellular component",
  "gene_symbol": "HMSD",
  "term_id": "UNKNOWN:0003",
  "gene_name": "Serpin-like protein HMSD",
  "gene": "UniProtKB:A8MTL9"
}